{
  "gene_name": "Somatoliberin",
  "gene_symbol": "GHRH",
  "gene": "UniProtKB:P01286",
  "term_label": "growth hormone-releasing hormone receptor binding",
  "term_id": "GO:0031770"
}